{
  "gene_name": "Endoribonuclease Dicer",
  "gene": "UniProtKB:Q9UPY3",
  "gene_symbol": "DICER1",
  "term_label": "deoxyribonuclease I activity",
  "term_id": "GO:0004530"
}